{
  "term_label": "chromatin",
  "gene_name": "Transcription factor 12",
  "gene": "UniProtKB:Q99081",
  "term_id": "GO:0000785",
  "gene_symbol": "TCF12"
}